{
  "gene_name": "Zinc finger protein 276",
  "gene": "UniProtKB:Q8N554",
  "term_label": "RNA polymerase II cis-regulatory region sequence-specific DNA binding",
  "term_id": "GO:0000978",
  "gene_symbol": "ZNF276"
}